{
  "gene_name": "Sulfate anion transporter 1",
  "term_label": "sulfate transmembrane transport",
  "gene": "UniProtKB:Q9H2B4",
  "term_id": "GO:1902358",
  "gene_symbol": "SLC26A1"
}